{
  "gene_name": "Ribose-phosphate pyrophosphokinase 2",
  "term_id": "GO:0006015",
  "term_label": "5-phosphoribose 1-diphosphate biosynthetic process",
  "gene": "UniProtKB:P11908",
  "gene_symbol": "PRPS2"
}